{
  "gene": "UniProtKB:P03999",
  "term_id": "GO:0071482",
  "term_label": "cellular response to light stimulus",
  "gene_name": "Short-wave-sensitive opsin 1",
  "gene_symbol": "OPN1SW"
}